calcineurin complex [GO:0005955] (cellular component) Also known as: protein phosphatase type 2B complex, calcium-dependent protein serine/threonine phosphatase complex Definition: A heterodimeric calcium ion and calmodulin dependent protein phosphatase composed of catalytic and regulatory subunits; the regulatory subunit is very similar in sequence to calmodulin. Relationships: is a type of protein serine/threonine phosphatase complex [GO:0008287]; is a type of intracellular protein-containing complex [GO:0140535] References: PMID:26794871